glucosamine metabolic process [GO:0006041] (biological process) Also known as: chitosamine metabolic process, chitosamine metabolism, glucosamine metabolism Subtypes: glucosamine biosynthetic process [GO:0006042], glucosamine catabolic process [GO:0006043] Definition: The chemical reactions and pathways involving glucosamine (2-amino-2-deoxyglucopyranose), an aminodeoxysugar that occurs in combined form in chitin. Sources: GOC:jl, ISBN:0198506732 Relationships: is a type of amino sugar metabolic process [GO:0006040]